neuronal dense core vesicle lumen [GO:0099013] (cellular component) Sources: GOC:dos Relationships: is a type of GO:0098898; is part of neuronal dense core vesicle [GO:0098992] Definition: The volume enclosed by a neuronal dense core vesicle membrane.